{
  "term_label": "cytoskeleton",
  "gene_name": "Keratin, type I cuticular Ha3-I",
  "gene_symbol": "KRT33A",
  "term_id": "GO:0005856",
  "gene": "UniProtKB:O76009"
}